{
  "term_id": "UNKNOWN:0001",
  "gene_name": "WD repeat domain-containing protein 83",
  "gene_symbol": "WDR83",
  "gene": "UniProtKB:Q9BRX9",
  "term_label": "Unknown molecular function"
}